{
  "term_id": "GO:0031507",
  "gene": "UniProtKB:P0DPK2",
  "gene_name": "Histone H3.Y",
  "term_label": "heterochromatin formation",
  "gene_symbol": "H3Y1"
}